response to nematode [GO:0009624] (biological process) Relationships: is a type of response to other organism [GO:0051707] Definition: Any process that results in a change in state or activity of a cell or an organism (in terms of movement, secretion, enzyme production, gene expression, etc.) as a result of a stimulus from a nematode. Sources: GOC:hb Also known as: response to nematodes